{
  "term_id": "GO:0005789",
  "term_label": "endoplasmic reticulum membrane",
  "gene_name": "Organic solute transporter subunit alpha",
  "gene": "UniProtKB:Q86UW1",
  "gene_symbol": "SLC51A"
}